{
  "gene_symbol": "UBE2B",
  "term_id": "GO:0000209",
  "term_label": "protein polyubiquitination",
  "gene": "UniProtKB:P63146",
  "gene_name": "Ubiquitin-conjugating enzyme E2 B"
}